lateral wall of outer hair cell [GO:0120249] (cellular component) Relationships: is_a lateral part of cell [GO:0097574] References: PMID:26352669, PMID:31920560, PMID:9412485 Sources: GOC:krc Also known as: outer hair cell lateral wall, OHC lateral wall, lateral wall of OHC Definition: The lateral wall of an outer hair cell (OHC) is a unique trilaminate composite consisting of the plasma membrane, an underlying cytoskeletal network containing an actin-spectrin cortical lattice, and an adjacent system of circumferential lamellar organelles known as the subsurface cisternae.